mitotic cell cycle [GO:0000278] (biological process) Definition: Progression through the phases of the mitotic cell cycle, the most common eukaryotic cell cycle, which canonically comprises four successive phases called G1, S, G2, and M and includes replication of the genome and the subsequent segregation of chromosomes into daughter cells. In some variant cell cycles nuclear replication or nuclear division may not be followed by cell division, or G1 and G2 phases may be absent. Regulation: regulated by regulation of mitotic cell cycle [GO:0007346]; negatively regulated by GO:0045930; positively regulated by positive regulation of mitotic cell cycle [GO:0045931] Also known as: mitosis Note: Note that this term should not be confused with 'GO:0140014 ; mitotic nuclear division'. 'GO:0000278 ; mitotic cell cycle represents the entire mitotic cell cycle, while 'GO:0140014 ; mitotic nuclear division' specifically represents the actual nuclear division step of the mitotic cell cycle. Sources: GOC:mah, ISBN:0815316194 Subtypes: endomitotic cell cycle [GO:0007113], second mitotic wave involved in compound eye morphogenesis [GO:0016330], cell cycle comprising mitosis without cytokinesis [GO:0033301], mitotic cell cycle, embryonic [GO:0045448] Relationships: is a type of GO:0007049; has part GO:0140014